{
  "gene": "UniProtKB:Q99470",
  "gene_symbol": "SDF2",
  "term_label": "Unknown molecular function",
  "term_id": "UNKNOWN:0001",
  "gene_name": "Stromal cell-derived factor 2"
}